{
  "term_label": "Unknown cellular component",
  "gene_name": "Pleckstrin homology domain-containing family G member 3",
  "gene": "UniProtKB:A1L390",
  "gene_symbol": "PLEKHG3",
  "term_id": "UNKNOWN:0003"
}